{
  "gene_name": "Autoimmune regulator",
  "term_label": "regulation of thymocyte migration",
  "gene": "UniProtKB:O43918",
  "gene_symbol": "AIRE",
  "term_id": "GO:2000410"
}